{
  "gene_symbol": "CNGA2",
  "term_label": "intracellularly cGMP-activated cation channel activity",
  "term_id": "GO:0005223",
  "gene": "UniProtKB:Q16280",
  "gene_name": "Cyclic nucleotide-gated olfactory channel"
}